{
  "term_id": "GO:0036064",
  "gene_symbol": "AHI1",
  "term_label": "ciliary basal body",
  "gene": "UniProtKB:Q8N157",
  "gene_name": "Jouberin"
}